{
  "term_label": "Unknown biological process",
  "gene_name": "Photoreceptor ankyrin repeat protein",
  "term_id": "UNKNOWN:0002",
  "gene_symbol": "ANKRD33",
  "gene": "UniProtKB:Q7Z3H0"
}